{
  "gene_symbol": "ZYG11A",
  "gene_name": "Protein zyg-11 homolog A",
  "term_id": "GO:0031462",
  "gene": "UniProtKB:Q6WRX3",
  "term_label": "Cul2-RING ubiquitin ligase complex"
}